{
  "term_label": "metalloendopeptidase activity",
  "term_id": "GO:0004222",
  "gene_symbol": "MMP19",
  "gene_name": "Matrix metalloproteinase-19",
  "gene": "UniProtKB:Q99542"
}